{
  "gene_name": "Probable ATP-dependent RNA helicase DDX60",
  "term_label": "defense response to virus",
  "term_id": "GO:0051607",
  "gene": "UniProtKB:Q8IY21",
  "gene_symbol": "DDX60"
}